protein C-terminal S-isoprenylcysteine carboxyl O-methyltransferase activity [GO:0004671] (molecular function) Sources: EC:2.1.1.100 Also known as: protein-S-isoprenylcysteine O-methyltransferase activity, S-adenosyl-L-methionine:protein-C-terminal-S-farnesyl-L-cysteine O-methyltransferase activity, S-farnesylcysteine methyltransferase activity, farnesyl cysteine C-terminal methyltransferase activity, farnesyl-protein carboxymethyltransferase activity, farnesylated protein C-terminal O-methyltransferase activity, isoprenylated protein methyltransferase activity, isoprenylcysteine carboxylmethyltransferase activity, prenylated protein carboxyl methyltransferase activity, prenylated protein methyltransferase activity, prenylcysteine carboxyl methyltransferase activity, prenylcysteine carboxylmethyltransferase activity, prenylcysteine carboxymethyltransferase activity, prenylcysteine methyltransferase activity, protein C-terminal farnesylcysteine O-methyltransferase activity, protein S-farnesylcysteine C-terminal methyltransferase activity Definition: Catalysis of the reaction: S-adenosyl-L-methionine + protein C-terminal S-farnesyl-L-cysteine = S-adenosyl-L-homocysteine + protein C-terminal S-farnesyl-L-cysteine methyl ester. Relationships: is a type of GO:0003880; is a type of S-adenosylmethionine-dependent methyltransferase activity [GO:0008757]